{
  "term_id": "UNKNOWN:0002",
  "gene_name": "Myb_SANT-like DNA-binding domain-containing protein 7",
  "gene_symbol": "MSANTD7",
  "term_label": "Unknown biological process",
  "gene": "UniProtKB:A0A1W2PQ72"
}